cellular response to interleukin-21 [GO:0098757] (biological process) Relationships: is a type of GO:0098756 Also known as: cellular response to IL-21 Sources: GOC:BHF, GOC:mah Definition: Any process that results in a change in state or activity of a cell (in terms of movement, secretion, enzyme production, gene expression, etc.) as a result of an interleukin-21 stimulus.